{
  "gene_name": "Calcineurin-binding protein cabin-1",
  "term_id": "GO:0031491",
  "gene": "UniProtKB:Q9Y6J0",
  "gene_symbol": "CABIN1",
  "term_label": "nucleosome binding"
}